establishment of mitotic spindle asymmetry [GO:0061867] (biological process) References: PMID:26659188 Relationships: is a type of mitotic spindle organization [GO:0007052] Definition: The mitotic spindle organization process by which a mitotic spindle becomes asymmetric either in position or structure.